{
  "gene": "UniProtKB:P47871",
  "gene_symbol": "GCGR",
  "term_label": "plasma membrane",
  "gene_name": "Glucagon receptor",
  "term_id": "GO:0005886"
}